positive regulation of erythrocyte aggregation [GO:0034120] (biological process) Also known as: positive regulation of RBC aggregation, positive regulation of red blood cell aggregation Sources: GOC:add Definition: Any process that activates or increases the frequency, rate, or extent of erythrocyte aggregation. Relationships: is a type of positive regulation of homotypic cell-cell adhesion [GO:0034112]; is a type of regulation of erythrocyte aggregation [GO:0034118]; positively regulates erythrocyte aggregation [GO:0034117]